{
  "term_id": "GO:0072659",
  "gene_name": "Protrudin",
  "term_label": "protein localization to plasma membrane",
  "gene": "UniProtKB:Q5T4F4",
  "gene_symbol": "ZFYVE27"
}